ligand-modulated transcription factor activity [GO:0098531] (molecular function) Definition: A DNA-binding transcription factor activity regulated by binding to a ligand and that modulates the transcription of specific genes and gene sets. Examples include the lac and trp repressors in E.coli and steroid hormone receptors. Subtypes: nuclear receptor activity [GO:0004879], GO:0141096, ligand-modulated transcription activator activity [GO:0141097] Also known as: direct ligand regulated sequence-specific DNA binding transcription factor activity, transcription factor activity, direct ligand regulated sequence-specific DNA binding, ligand-activated transcription factor activity Relationships: is a type of DNA-binding transcription factor activity [GO:0003700] References: PMID:25568920, PMID:8735275 Sources: GOC:dos Note: For usage guidance, see comment in GO:0003700 ; DNA-binding transcription factor activity.